polysaccharide catabolic process [GO:0000272] (biological process) References: PMID:33139480 Also known as: polysaccharide breakdown, polysaccharide catabolism, polysaccharide degradation, multicellular organismal polysaccharide catabolic process Subtypes: glucan catabolic process [GO:0009251], fructan catabolic process [GO:0010147], cell septum edging catabolic process [GO:0030995], GO:0031222, GO:0033393, GO:0042122, cell wall polysaccharide catabolic process [GO:0044347], pectin catabolic process [GO:0045490], galactomannan catabolic process [GO:0051682], alpha-linked polysaccharide catabolism to maltotriose [GO:0052786], alpha-linked polysaccharide catabolism to maltopentaose [GO:0052787], GO:0093001, mannogen catabolic process [GO:0106305], glucomannan catabolic process [GO:2000884], galactoglucomannan catabolic process [GO:2000885], hemicellulose catabolic process [GO:2000895] Definition: The chemical reactions and pathways resulting in the breakdown of a polysaccharide, a polymer of many (typically more than 10) monosaccharide residues linked glycosidically. Relationships: is a type of polysaccharide metabolic process [GO:0005976]; is a type of macromolecule catabolic process [GO:0009057]; is a type of GO:0016052